{
  "term_id": "GO:0061844",
  "gene": "UniProtKB:O00585",
  "term_label": "antimicrobial humoral immune response mediated by antimicrobial peptide",
  "gene_symbol": "CCL21",
  "gene_name": "C-C motif chemokine 21"
}